{
  "gene_symbol": "CEBPG",
  "gene_name": "CCAAT_enhancer-binding protein gamma",
  "term_label": "regulation of transcription by RNA polymerase II",
  "gene": "UniProtKB:P53567",
  "term_id": "GO:0006357"
}